{
  "gene_name": "T cell receptor alpha joining 57 (Fragment)",
  "gene": "UniProtKB:A0A075B704",
  "term_id": "UNKNOWN:0002",
  "gene_symbol": "TRAJ57",
  "term_label": "Unknown biological process"
}